{
  "gene_name": "Nucleoprotein TPR",
  "gene_symbol": "TPR",
  "gene": "UniProtKB:P12270",
  "term_label": "nuclear pore",
  "term_id": "GO:0005643"
}